{
  "gene_name": "Tubulin alpha-1C chain",
  "gene_symbol": "TUBA1C",
  "gene": "UniProtKB:Q9BQE3",
  "term_label": "cytoplasm",
  "term_id": "GO:0005737"
}